{
  "gene_name": "Vasoactive intestinal polypeptide receptor 1",
  "term_label": "plasma membrane",
  "gene": "UniProtKB:P32241",
  "gene_symbol": "VIPR1",
  "term_id": "GO:0005886"
}